RNA polymerase III promoter clearance [GO:0001110] (biological process) Sources: GOC:txnOH Also known as: promoter clearance from RNA polymerase III promoter Relationships: is a type of promoter clearance during DNA-templated transcription [GO:0001109]; is part of GO:0006383 Definition: A process that mediates the transition from the initiation to the elongation phases of transcription by RNA polymerase III, generally including a conformational change from the initiation conformation to the elongation conformation. Promoter clearance often involves breaking contact with transcription factors involved only in the initiation phase.